{
  "term_id": "GO:0050839",
  "gene_symbol": "PCDHA13",
  "gene_name": "Protocadherin alpha-13",
  "gene": "UniProtKB:Q9Y5I0",
  "term_label": "cell adhesion molecule binding"
}